isoprenoid catabolic process [GO:0008300] (BP) Relationships: is a type of isoprenoid metabolic process [GO:0006720]; is a type of GO:0016042 Definition: The chemical reactions and pathways resulting in the breakdown of an isoprenoid compound, isoprene (2-methylbuta-1,3-diene) or compounds containing or derived from linked isoprene (3-methyl-2-butenylene) residues. Subtypes: prenol catabolic process [GO:0016092], GO:0016095, terpenoid catabolic process [GO:0016115], apocarotenoid catabolic process [GO:0043290], terpene catabolic process [GO:0046247] Sources: ISBN:0198506732 Also known as: isoprenoid breakdown, isoprenoid catabolism, isoprenoid degradation, polyisoprenoid breakdown, polyisoprenoid catabolic process, polyisoprenoid catabolism, polyisoprenoid degradation, polyterpene catabolic process, polyterpene catabolism